{
  "term_id": "GO:0006357",
  "gene": "UniProtKB:P51449",
  "gene_symbol": "RORC",
  "gene_name": "Nuclear receptor ROR-gamma",
  "term_label": "regulation of transcription by RNA polymerase II"
}